{
  "gene_symbol": "ACVR1",
  "term_label": "SMAD binding",
  "term_id": "GO:0046332",
  "gene_name": "Activin receptor type-1",
  "gene": "UniProtKB:Q04771"
}